{
  "gene_symbol": "PLK5",
  "gene": "UniProtKB:Q496M5",
  "gene_name": "Inactive serine_threonine-protein kinase PLK5",
  "term_label": "cytoplasm",
  "term_id": "GO:0005737"
}